{
  "term_id": "GO:0005886",
  "gene_name": "5-hydroxytryptamine receptor 1E",
  "term_label": "plasma membrane",
  "gene": "UniProtKB:P28566",
  "gene_symbol": "HTR1E"
}